positive regulation of nuclear-transcribed mRNA catabolic process, deadenylation-dependent decay [GO:1900153] (biological process) Sources: GOC:TermGenie, GOC:mcc Also known as: positive regulation of deadenylation-dependent mRNA decay, positive regulation of mRNA breakdown, deadenylation-dependent decay, positive regulation of mRNA catabolic process, deadenylation-dependent, positive regulation of mRNA catabolic process, deadenylylation-dependent, positive regulation of mRNA catabolism, deadenylation-dependent, positive regulation of mRNA catabolism, deadenylylation-dependent, positive regulation of mRNA degradation, deadenylation-dependent decay, positive regulation of nuclear mRNA catabolic process, deadenylation-dependent decay, up regulation of deadenylation-dependent mRNA decay, up regulation of mRNA breakdown, deadenylation-dependent decay, up regulation of mRNA catabolic process, deadenylation-dependent, up regulation of mRNA catabolic process, deadenylylation-dependent, up regulation of mRNA catabolism, deadenylation-dependent, up regulation of mRNA catabolism, deadenylylation-dependent, up regulation of mRNA degradation, deadenylation-dependent decay, up regulation of nuclear mRNA catabolic process, deadenylation-dependent decay, up regulation of nuclear-transcribed mRNA catabolic process, deadenylation-dependent decay, up-regulation of deadenylation-dependent mRNA decay, up-regulation of mRNA breakdown, deadenylation-dependent decay, up-regulation of mRNA catabolic process, deadenylation-dependent, up-regulation of mRNA catabolic process, deadenylylation-dependent, up-regulation of mRNA catabolism, deadenylation-dependent, up-regulation of mRNA catabolism, deadenylylation-dependent, up-regulation of mRNA degradation, deadenylation-dependent decay, up-regulation of nuclear mRNA catabolic process, deadenylation-dependent decay, up-regulation of nuclear-transcribed mRNA catabolic process, deadenylation-dependent decay, upregulation of deadenylation-dependent mRNA decay, upregulation of mRNA breakdown, deadenylation-dependent decay, upregulation of mRNA catabolic process, deadenylation-dependent, upregulation of mRNA catabolic process, deadenylylation-dependent, upregulation of mRNA catabolism, deadenylation-dependent, upregulation of mRNA catabolism, deadenylylation-dependent, upregulation of mRNA degradation, deadenylation-dependent decay, upregulation of nuclear mRNA catabolic process, deadenylation-dependent decay, upregulation of nuclear-transcribed mRNA catabolic process, deadenylation-dependent decay, activation of deadenylation-dependent mRNA decay, activation of mRNA breakdown, deadenylation-dependent decay, activation of mRNA catabolic process, deadenylation-dependent, activation of mRNA catabolic process, deadenylylation-dependent, activation of mRNA catabolism, deadenylation-dependent, activation of mRNA catabolism, deadenylylation-dependent, activation of mRNA degradation, deadenylation-dependent decay, activation of nuclear mRNA catabolic process, deadenylation-dependent decay, activation of nuclear-transcribed mRNA catabolic process, deadenylation-dependent decay Definition: Any process that activates or increases the frequency, rate or extent of nuclear-transcribed mRNA catabolic process, deadenylation-dependent decay. Relationships: is_a positive regulation of mRNA catabolic process [GO:0061014]; is a type of GO:1900151; RO_0002213 nuclear-transcribed mRNA catabolic process, deadenylation-dependent decay [GO:0000288]